3,4-dihydroxybenzoate biosynthetic process [GO:0046279] (biological process) Relationships: is a type of catechol-containing compound biosynthetic process [GO:0009713]; is a type of GO:0046278; is a type of monocarboxylic acid biosynthetic process [GO:0072330] Sources: GOC:ai Also known as: protocatechuate anabolism, protocatechuate biosynthesis, protocatechuate biosynthetic process, protocatechuate formation, protocatechuate synthesis Definition: The chemical reactions and pathways resulting in the formation of 3,4-dihydroxybenzoate.